{
  "gene_name": "Zinc finger protein 704",
  "gene": "UniProtKB:Q6ZNC4",
  "term_id": "GO:0000978",
  "gene_symbol": "ZNF704",
  "term_label": "RNA polymerase II cis-regulatory region sequence-specific DNA binding"
}